{
  "term_label": "zinc ion transmembrane transporter activity",
  "gene": "UniProtKB:Q9Y6M5",
  "gene_name": "Proton-coupled zinc antiporter SLC30A1",
  "term_id": "GO:0005385",
  "gene_symbol": "SLC30A1"
}